{
  "gene_name": "Zinc finger MYM-type protein 5",
  "gene": "UniProtKB:Q9UJ78",
  "gene_symbol": "ZMYM5",
  "term_id": "UNKNOWN:0002",
  "term_label": "Unknown biological process"
}